{
  "gene_symbol": "LARS1",
  "term_label": "Unknown cellular component",
  "gene_name": "Leucine--tRNA ligase, cytoplasmic",
  "gene": "UniProtKB:Q9P2J5",
  "term_id": "UNKNOWN:0003"
}